{
  "gene_name": "Thyrotropin subunit beta",
  "term_label": "hormone activity",
  "gene_symbol": "TSHB",
  "gene": "UniProtKB:P01222",
  "term_id": "GO:0005179"
}